cap-dependent translational initiation [GO:0002191] (biological process) References: PMID:17284590, PMID:19604130 Relationships: is a type of cytoplasmic translational initiation [GO:0002183]; has part GO:0160296 Regulation: regulated by regulation of cap-dependent translational initiation [GO:1903674]; negatively regulated by GO:1903675; positively regulated by positive regulation of cap-dependent translational initiation [GO:1903676] Definition: The process where the cap structure, composed of a 7- methylguanosine (m7G) group and associated cap-binding proteins, located at the 5' end of an mRNA molecule, which serves as a molecular tag that marks the spot where the 40S ribosomal subunit, is recruited and will then scan in a 5' to 3' direction until an AUG codon is encountered in an appropriate sequence context to initiate mRNA translation.